{
  "term_label": "plasma membrane",
  "term_id": "GO:0005886",
  "gene": "UniProtKB:Q6IF42",
  "gene_name": "Olfactory receptor 2A2",
  "gene_symbol": "OR2A2"
}